cyclodextrin metabolic process [GO:2000900] (biological process) Definition: The chemical reactions and pathways involving a cyclodextrin. Sources: GOC:mengo_curators Also known as: cyclodextrin metabolism Relationships: is a type of GO:0009311; is a type of glucan metabolic process [GO:0044042] Subtypes: cyclodextrin catabolic process [GO:2000901]